{
  "term_id": "GO:0045944",
  "gene_name": "Single-stranded DNA-binding protein 2",
  "gene_symbol": "SSBP2",
  "gene": "UniProtKB:P81877",
  "term_label": "positive regulation of transcription by RNA polymerase II"
}